L-pipecolate oxidase activity [GO:0050031] (molecular function) Sources: EC:1.5.3.7, RHEA:11992 Definition: Catalysis of the reaction: L-pipecolate + O2 = 2,3,4,5-tetrahydropyridine-2-carboxylate + H2O2 + H+. Delta1-piperideine-6-carboxylate is also known as 2,3,4,5-tetrahydropyridine-2-carboxylate. Also known as: L-pipecolate:oxygen 1,6-oxidoreductase activity, L-pipecolic acid oxidase activity Relationships: is a type of oxidoreductase activity, acting on the CH-NH group of donors, oxygen as acceptor [GO:0016647]